{
  "term_label": "cytoplasmic exosome (RNase complex)",
  "gene_name": "DIS3-like exonuclease 1",
  "term_id": "GO:0000177",
  "gene": "UniProtKB:Q8TF46",
  "gene_symbol": "DIS3L"
}